{
  "term_label": "Unknown molecular function",
  "term_id": "UNKNOWN:0001",
  "gene_symbol": "ATP6V1B2",
  "gene": "UniProtKB:P21281",
  "gene_name": "V-type proton ATPase subunit B, brain isoform"
}